L-tryptophan transmembrane transport [GO:1904556] (BP) Relationships: is a type of tryptophan transport [GO:0015827]; is_a L-alpha-amino acid transmembrane transport [GO:1902475] Definition: The directed movement of L-tryptophan across a membrane. Subtypes: L-tryptophan import across plasma membrane [GO:1904272] Sources: GOC:TermGenie, GOC:kmv, GO_REF:0000069